negative regulation of keratinocyte migration [GO:0051548] (biological process) Definition: Any process that stops, prevents, or reduces the frequency, rate or extent of keratinocyte migration. Relationships: is a type of GO:0010633; is a type of regulation of keratinocyte migration [GO:0051547]; RO_0002212 keratinocyte migration [GO:0051546] Also known as: down regulation of keratinocyte migration, down-regulation of keratinocyte migration, downregulation of keratinocyte migration, inhibition of keratinocyte migration Sources: GOC:ai